{
  "gene_name": "E3 SUMO-protein ligase PIAS3",
  "term_id": "GO:0000785",
  "gene_symbol": "PIAS3",
  "term_label": "chromatin",
  "gene": "UniProtKB:Q9Y6X2"
}